{
  "gene_symbol": "ZNF746",
  "term_id": "GO:0000978",
  "term_label": "RNA polymerase II cis-regulatory region sequence-specific DNA binding",
  "gene_name": "Zinc finger protein 746",
  "gene": "UniProtKB:Q6NUN9"
}